positive regulation of glycolytic fermentation to ethanol [GO:2001172] (biological process) Definition: Any process that activates or increases the frequency, rate or extent of glucose catabolic process to ethanol. Sources: GOC:obol Also known as: positive regulation of ethanol fermentation, positive regulation of glucose fermentation to ethanol Relationships: is a type of positive regulation of catabolic process [GO:0009896]; is a type of positive regulation of small molecule metabolic process [GO:0062013]; is_a regulation of glycolytic fermentation to ethanol [GO:2001154]; positively regulates pyruvate fermentation to ethanol [GO:0019655]